{
  "gene_symbol": "LINC00587",
  "gene": "UniProtKB:B1AMM8",
  "gene_name": "Putative uncharacterized protein encoded by LINC00587",
  "term_label": "Unknown biological process",
  "term_id": "UNKNOWN:0002"
}